vitamin D metabolic process [GO:0042359] (biological process) Relationships: is a type of steroid metabolic process [GO:0008202] Sources: GOC:mah, ISBN:0471331309 Definition: The chemical reactions and pathways involving vitamin D, any of a group of related, fat-soluble compounds that are derived from delta-5,7 steroids and play a central role in calcium metabolism. Specific forms of vitamin D include calciferol (ergocalciferol; vitamin D2) and cholecalciferol (calciol; vitamin D3). Also known as: vitamin D metabolism, calciferol metabolic process, calciferol metabolism, cholecalciferol metabolic process, cholecalciferol metabolism, ergocalciferol metabolic process, ergocalciferol metabolism Subtypes: vitamin D biosynthetic process [GO:0042368], vitamin D catabolic process [GO:0042369], vitamin D3 metabolic process [GO:0070640]